{
  "term_label": "carnitine O-palmitoyltransferase activity",
  "gene": "UniProtKB:Q92523",
  "gene_name": "Carnitine O-palmitoyltransferase 1, muscle isoform",
  "gene_symbol": "CPT1B",
  "term_id": "GO:0004095"
}